methanol oxidation [GO:0015946] (biological process) Definition: The chemical reactions and pathways resulting in the conversion of methanol to methyl-Coenzyme M. Relationships: is a type of methanol metabolic process [GO:0015945] Sources: MetaCyc:CO2FORM-PWY